phosphomannomutase activity [GO:0004615] (molecular function) Relationships: is a type of intramolecular phosphotransferase activity [GO:0016868] Definition: Catalysis of the reaction: alpha-D-mannose 1-phosphate = D-mannose 6-phosphate. Also known as: D-mannose 1,6-phosphomutase activity, alpha-D-mannose 1,6-phosphomutase activity, mannose phosphomutase activity, phosphomannose mutase activity Sources: EC:5.4.2.8, RHEA:11140